{
  "gene": "UniProtKB:Q76EJ3",
  "gene_symbol": "SLC35D2",
  "gene_name": "UDP-N-acetylglucosamine_UDP-glucose_GDP-mannose transporter",
  "term_label": "UDP-glucuronate transmembrane transporter activity",
  "term_id": "GO:0005461"
}